interleukin-33 receptor activity [GO:0002114] (molecular function) Relationships: is a type of cytokine receptor activity [GO:0004896]; is part of interleukin-33-mediated signaling pathway [GO:0038172]; has part interleukin-33 binding [GO:0002113] Also known as: IL-33 receptor activity, IL-33R Definition: Combining with interleukin-33 and transmitting the signal from one side of the membrane to the other to initiate a change in cell activity. Sources: GOC:hjd, GOC:signaling